glycine-tRNA ligase activity [GO:0004820] (molecular function) Sources: EC:6.1.1.14 Definition: Catalysis of the reaction: ATP + glycine + tRNA(Gly) = AMP + diphosphate + glycyl-tRNA(Gly). Also known as: glycyl-tRNA synthetase activity, glycine:tRNAGly ligase (AMP-forming) activity, glycyl translase activity, glycyl-transfer RNA synthetase activity, glycyl-transfer ribonucleate synthetase activity, glycyl-transfer ribonucleic acid synthetase activity Relationships: is a type of aminoacyl-tRNA ligase activity [GO:0004812]